{
  "term_id": "GO:0042391",
  "gene_symbol": "HTR3C",
  "gene_name": "5-hydroxytryptamine receptor 3C",
  "gene": "UniProtKB:Q8WXA8",
  "term_label": "regulation of membrane potential"
}